{
  "gene_symbol": "INPP5J",
  "gene": "UniProtKB:Q15735",
  "term_label": "ruffle",
  "gene_name": "Phosphatidylinositol 4,5-bisphosphate 5-phosphatase A",
  "term_id": "GO:0001726"
}